{
  "term_id": "GO:0005768",
  "gene_symbol": "CLVS1",
  "term_label": "endosome",
  "gene_name": "Clavesin-1",
  "gene": "UniProtKB:Q8IUQ0"
}